{
  "term_id": "UNKNOWN:0002",
  "gene": "UniProtKB:A2VCK2",
  "gene_name": "Doublecortin domain-containing protein 2B",
  "gene_symbol": "DCDC2B",
  "term_label": "Unknown biological process"
}